{
  "term_label": "transcription factor TFIIIB complex",
  "gene_symbol": "BDP1",
  "gene": "UniProtKB:A6H8Y1",
  "term_id": "GO:0000126",
  "gene_name": "Transcription factor TFIIIB component B'' homolog"
}